hydroxypyruvate isomerase activity [GO:0008903] (molecular function) Relationships: is a type of intramolecular oxidoreductase activity, interconverting aldoses and ketoses [GO:0016861] Sources: EC:5.3.1.22, RHEA:11952 Definition: Catalysis of the reaction: 3-hydroxypyruvate = 2-hydroxy-3-oxopropanoate. Also known as: hydroxypyruvate aldose-ketose-isomerase activity, hydroxypyruvate ketol-isomerase activity